{
  "gene_symbol": "BCAR1",
  "term_id": "GO:0005886",
  "term_label": "plasma membrane",
  "gene": "UniProtKB:P56945",
  "gene_name": "Breast cancer anti-estrogen resistance protein 1"
}